{
  "gene_name": "Low-density lipoprotein receptor-related protein 1B",
  "gene_symbol": "LRP1B",
  "gene": "UniProtKB:Q9NZR2",
  "term_id": "GO:0043235",
  "term_label": "receptor complex"
}